positive regulation of protein modification process [GO:0031401] (biological process) Also known as: up regulation of protein modification, up-regulation of protein modification, upregulation of protein modification, activation of protein modification, stimulation of protein modification Subtypes: positive regulation of protein phosphorylation [GO:0001934], positive regulation of protein glutathionylation [GO:0010733], positive regulation of protein deacetylation [GO:0090312], GO:1900724, positive regulation of post-translational protein modification [GO:1901875], positive regulation of protein acetylation [GO:1901985], positive regulation of protein lipidation [GO:1903061], positive regulation of protein polyglycylation [GO:1903346], GO:1904287, positive regulation of protein oxidation [GO:1904808], positive regulation of peptidyl-cysteine S-nitrosylation [GO:2000170], GO:2000541 Sources: GOC:mah, GOC:tb Definition: Any process that activates or increases the frequency, rate or extent of the covalent alteration of one or more amino acid residues within a protein. Relationships: is a type of regulation of protein modification process [GO:0031399]; is a type of positive regulation of protein metabolic process [GO:0051247]; positively regulates protein modification process [GO:0036211]